{
  "gene_name": "Zinc finger and SCAN domain-containing protein 32",
  "gene_symbol": "ZSCAN32",
  "term_id": "GO:0006357",
  "term_label": "regulation of transcription by RNA polymerase II",
  "gene": "UniProtKB:Q9NX65"
}